peripheral B cell receptor editing [GO:0002345] (biological process) Definition: The process that takes place mainly in germinal center B cells in which a large number of mutations are generated in the heavy chain and light chain V-region genes and their immediately surrounding introns in order to increase antibody diversity and contribute to affinity maturation. Relationships: is a type of B cell receptor editing [GO:0002452] Sources: GOC:jal Also known as: peripheral B lymphocyte receptor editing, peripheral B-cell receptor editing, peripheral B-lymphocyte receptor editing